{
  "term_label": "actin cytoskeleton organization",
  "gene_symbol": "LIMK2",
  "gene": "UniProtKB:P53671",
  "gene_name": "LIM domain kinase 2",
  "term_id": "GO:0030036"
}